{
  "term_label": "ubiquitin-like ligase-substrate adaptor activity",
  "gene_name": "F-box only protein 42",
  "term_id": "GO:1990756",
  "gene": "UniProtKB:Q6P3S6",
  "gene_symbol": "FBXO42"
}